negative regulation of compound eye photoreceptor development [GO:0045316] (biological process) Definition: Any process that stops, prevents, or reduces the frequency, rate or extent of compound eye photoreceptor development. Relationships: is a type of negative regulation of eye photoreceptor cell development [GO:0042480]; is a type of regulation of compound eye photoreceptor development [GO:0045314]; RO_0002212 compound eye photoreceptor development [GO:0042051] Sources: GOC:bf Also known as: down regulation of eye photoreceptor development, down-regulation of eye photoreceptor development, downregulation of eye photoreceptor development, inhibition of eye photoreceptor development, negative regulation of eye photoreceptor development